{
  "gene_name": "Zinc finger C4H2 domain-containing protein",
  "gene_symbol": "ZC4H2",
  "term_label": "Unknown molecular function",
  "gene": "UniProtKB:Q9NQZ6",
  "term_id": "UNKNOWN:0001"
}